{
  "term_id": "UNKNOWN:0003",
  "gene_name": "Maternal embryonic leucine zipper kinase",
  "term_label": "Unknown cellular component",
  "gene_symbol": "MELK",
  "gene": "UniProtKB:Q14680"
}